{
  "term_id": "GO:1902110",
  "term_label": "positive regulation of mitochondrial membrane permeability involved in apoptotic process",
  "gene_name": "O(6)-methylguanine-induced apoptosis 2",
  "gene_symbol": "STPG1",
  "gene": "UniProtKB:Q5TH74"
}